{
  "gene_symbol": "SYT7",
  "gene": "UniProtKB:O43581",
  "gene_name": "Synaptotagmin-7",
  "term_label": "plasma membrane",
  "term_id": "GO:0005886"
}